{
  "gene_symbol": "WDR12",
  "term_label": "maturation of 5.8S rRNA from tricistronic rRNA transcript (SSU-rRNA, 5.8S rRNA, LSU-rRNA)",
  "gene_name": "Ribosome biogenesis protein WDR12",
  "term_id": "GO:0000466",
  "gene": "UniProtKB:Q9GZL7"
}